{
  "term_id": "GO:0045259",
  "gene": "UniProtKB:P00846",
  "term_label": "proton-transporting ATP synthase complex",
  "gene_name": "ATP synthase subunit a",
  "gene_symbol": "MT-ATP6"
}